{
  "gene_name": "Elongation factor 1-gamma",
  "term_label": "cytoplasm",
  "gene_symbol": "EEF1G",
  "gene": "UniProtKB:P26641",
  "term_id": "GO:0005737"
}